Sertoli cell barrier remodeling [GO:0061843] (biological process) Definition: The tissue remodeling process by which the Sertoli cell barrier is temporarily disrupted and reorganized to accommodate the transit of preleptotene spermatocytes at stage VIII of the epithelial cycle. References: PMID:20534520, PMID:24467744 Relationships: is a type of tissue remodeling [GO:0048771] Also known as: blood testis barrier restructuring, restructuring of BTB, restructuring of blood-testis barrier, SCB remodeling, Sertoli cell barrier remodelling, Sertoli cell barrier restructuring, restructuring of SCB